heparanase complex [GO:1904974] (cellular component) Relationships: is a type of catalytic complex [GO:1902494] References: PMID:12927802 Sources: GOC:TermGenie, GOC:bhm, GO_REF:0000088 Definition: A protein complex which is capable of heparanase activity. Also known as: HEPS complex Note: An example of this is HPSE in human (Q9Y251) in PMID:12927802 (inferred from direct assay).